{
  "term_id": "GO:0030141",
  "gene": "UniProtKB:Q9UKQ9",
  "gene_symbol": "KLK9",
  "gene_name": "Kallikrein-9",
  "term_label": "secretory granule"
}